{
  "gene_symbol": "PLA2G12A",
  "term_id": "UNKNOWN:0003",
  "term_label": "Unknown cellular component",
  "gene_name": "Group XIIA secretory phospholipase A2",
  "gene": "UniProtKB:Q9BZM1"
}